{
  "gene_name": "BMP_retinoic acid-inducible neural-specific protein 1",
  "term_label": "cellular response to retinoic acid",
  "term_id": "GO:0071300",
  "gene": "UniProtKB:O60477",
  "gene_symbol": "BRINP1"
}